{
  "gene_name": "Protein SOGA3",
  "gene_symbol": "SOGA3",
  "term_id": "UNKNOWN:0002",
  "term_label": "Unknown biological process",
  "gene": "UniProtKB:Q5TF21"
}